{
  "gene_name": "Melanoma-associated antigen 3",
  "gene_symbol": "MAGEA3",
  "term_id": "GO:0042826",
  "gene": "UniProtKB:P43357",
  "term_label": "histone deacetylase binding"
}